{
  "term_label": "Cdc73/Paf1 complex",
  "gene_symbol": "CTR9",
  "gene": "UniProtKB:Q6PD62",
  "term_id": "GO:0016593",
  "gene_name": "RNA polymerase-associated protein CTR9 homolog"
}